{
  "term_id": "GO:0004864",
  "gene_symbol": "PPP1R2B",
  "gene": "UniProtKB:Q6NXS1",
  "gene_name": "Protein phosphatase inhibitor 2 family member B",
  "term_label": "protein phosphatase inhibitor activity"
}